{
  "term_label": "Unknown molecular function",
  "term_id": "UNKNOWN:0001",
  "gene": "UniProtKB:A0A2R8Y7Y5",
  "gene_name": "Protein CIST1",
  "gene_symbol": "CIST1"
}